{
  "term_id": "GO:0048306",
  "gene_name": "Protein S100-A7",
  "gene_symbol": "S100A7",
  "term_label": "calcium-dependent protein binding",
  "gene": "UniProtKB:P31151"
}